{
  "gene_name": "T cell receptor alpha variable 12-2",
  "term_id": "UNKNOWN:0002",
  "gene": "UniProtKB:A0A075B6T6",
  "gene_symbol": "TRAV12-2",
  "term_label": "Unknown biological process"
}